{
  "gene_symbol": "CYP26A1",
  "gene": "UniProtKB:O43174",
  "term_id": "GO:0007417",
  "gene_name": "Cytochrome P450 26A1",
  "term_label": "central nervous system development"
}